{
  "gene_name": "Runt-related transcription factor 1",
  "gene": "UniProtKB:Q01196",
  "term_id": "GO:0000978",
  "gene_symbol": "RUNX1",
  "term_label": "RNA polymerase II cis-regulatory region sequence-specific DNA binding"
}